positive regulation of protein processing in phagocytic vesicle [GO:1903923] (BP) Relationships: is a type of positive regulation of protein processing [GO:0010954]; is a type of regulation of protein processing in phagocytic vesicle [GO:1903921]; positively regulates GO:1900756 Definition: Any process that activates or increases the frequency, rate or extent of protein processing in phagocytic vesicle. Also known as: positive regulation of protein maturation by peptide bond cleavage in phagocytic vesicle, positive regulation of protein maturation by peptide bond cleavage in phagosome, positive regulation of protein maturation by peptide bond hydrolysis in phagocytic vesicle, positive regulation of protein maturation by peptide bond hydrolysis in phagosome, positive regulation of protein processing in phagosome, up regulation of protein maturation by peptide bond cleavage in phagocytic vesicle, up regulation of protein maturation by peptide bond cleavage in phagosome, up regulation of protein maturation by peptide bond hydrolysis in phagocytic vesicle, up regulation of protein maturation by peptide bond hydrolysis in phagosome, up regulation of protein processing in phagocytic vesicle, up regulation of protein processing in phagosome, up-regulation of protein maturation by peptide bond cleavage in phagocytic vesicle, up-regulation of protein maturation by peptide bond cleavage in phagosome, up-regulation of protein maturation by peptide bond hydrolysis in phagocytic vesicle, up-regulation of protein maturation by peptide bond hydrolysis in phagosome, up-regulation of protein processing in phagocytic vesicle, up-regulation of protein processing in phagosome, upregulation of protein maturation by peptide bond cleavage in phagocytic vesicle, upregulation of protein maturation by peptide bond cleavage in phagosome, upregulation of protein maturation by peptide bond hydrolysis in phagocytic vesicle, upregulation of protein maturation by peptide bond hydrolysis in phagosome, upregulation of protein processing in phagocytic vesicle, upregulation of protein processing in phagosome, activation of protein maturation by peptide bond cleavage in phagocytic vesicle, activation of protein maturation by peptide bond cleavage in phagosome, activation of protein maturation by peptide bond hydrolysis in phagocytic vesicle, activation of protein maturation by peptide bond hydrolysis in phagosome, activation of protein processing in phagocytic vesicle, activation of protein processing in phagosome, activation of peptidolysis during protein maturation in phagocytic vesicle, activation of peptidolysis during protein maturation in phagosome, activation of protein maturation by proteolysis in phagocytic vesicle, activation of protein maturation by proteolysis in phagosome, positive regulation of peptidolysis during protein maturation in phagocytic vesicle, positive regulation of peptidolysis during protein maturation in phagosome, positive regulation of protein maturation by proteolysis in phagocytic vesicle, positive regulation of protein maturation by proteolysis in phagosome, up regulation of peptidolysis during protein maturation in phagocytic vesicle, up regulation of peptidolysis during protein maturation in phagosome, up regulation of protein maturation by proteolysis in phagocytic vesicle, up regulation of protein maturation by proteolysis in phagosome, up-regulation of peptidolysis during protein maturation in phagocytic vesicle, up-regulation of peptidolysis during protein maturation in phagosome, up-regulation of protein maturation by proteolysis in phagocytic vesicle, up-regulation of protein maturation by proteolysis in phagosome, upregulation of peptidolysis during protein maturation in phagocytic vesicle, upregulation of peptidolysis during protein maturation in phagosome, upregulation of protein maturation by proteolysis in phagocytic vesicle, upregulation of protein maturation by proteolysis in phagosome References: PMID:23325791 Sources: GOC:TermGenie, GOC:als, GO_REF:0000058